{
  "gene_symbol": "FBXL4",
  "term_id": "GO:0019005",
  "gene_name": "F-box_LRR-repeat protein 4",
  "gene": "UniProtKB:Q9UKA2",
  "term_label": "SCF ubiquitin ligase complex"
}